{
  "gene_name": "Hepatic sodium_bile acid cotransporter",
  "term_label": "Unknown cellular component",
  "gene_symbol": "SLC10A1",
  "gene": "UniProtKB:Q14973",
  "term_id": "UNKNOWN:0003"
}